negative regulation of inositol biosynthetic process [GO:1900089] (biological process) Definition: Any process that stops, prevents or reduces the frequency, rate or extent of inositol biosynthetic process. Also known as: down regulation of inositol anabolism, down regulation of inositol biosynthesis, down regulation of inositol biosynthetic process, down regulation of inositol formation, down regulation of inositol synthesis, down regulation of vitamin Bh biosynthesis, down regulation of vitamin Bh biosynthetic process, down-regulation of inositol anabolism, down-regulation of inositol biosynthesis, down-regulation of inositol biosynthetic process, down-regulation of inositol formation, down-regulation of inositol synthesis, down-regulation of vitamin Bh biosynthesis, down-regulation of vitamin Bh biosynthetic process, downregulation of inositol anabolism, downregulation of inositol biosynthesis, downregulation of inositol biosynthetic process, downregulation of inositol formation, downregulation of inositol synthesis, downregulation of vitamin Bh biosynthesis, downregulation of vitamin Bh biosynthetic process, inhibition of inositol anabolism, inhibition of inositol biosynthesis, inhibition of inositol formation, inhibition of inositol synthesis, inhibition of vitamin Bh biosynthesis, inhibition of vitamin Bh biosynthetic process, negative regulation of inositol anabolism, negative regulation of inositol biosynthesis, negative regulation of inositol formation, negative regulation of inositol synthesis, negative regulation of vitamin Bh biosynthesis, negative regulation of vitamin Bh biosynthetic process, down regulation of myo-inositol biosynthesis, down regulation of myo-inositol biosynthetic process, down-regulation of myo-inositol biosynthesis, down-regulation of myo-inositol biosynthetic process, downregulation of myo-inositol biosynthesis, downregulation of myo-inositol biosynthetic process, inhibition of inositol biosynthetic process, inhibition of myo-inositol biosynthesis, inhibition of myo-inositol biosynthetic process, negative regulation of myo-inositol biosynthesis, negative regulation of myo-inositol biosynthetic process References: PMID:22307851 Sources: GOC:TermGenie Relationships: is a type of regulation of inositol biosynthetic process [GO:1900088]; is a type of GO:1902931; negatively regulates inositol biosynthetic process [GO:0006021]